{
  "gene_name": "Zinc finger protein 541",
  "gene": "UniProtKB:Q9H0D2",
  "term_label": "transcription corepressor activity",
  "gene_symbol": "ZNF541",
  "term_id": "GO:0003714"
}